{
  "gene_name": "Calpain-3",
  "term_label": "negative regulation of apoptotic process",
  "gene": "UniProtKB:P20807",
  "gene_symbol": "CAPN3",
  "term_id": "GO:0043066"
}